{
  "term_label": "plasma membrane",
  "gene_name": "Serotransferrin",
  "gene_symbol": "TF",
  "term_id": "GO:0005886",
  "gene": "UniProtKB:P02787"
}